{
  "term_id": "GO:0000122",
  "gene_symbol": "GLIS2",
  "gene_name": "Zinc finger protein GLIS2",
  "gene": "UniProtKB:Q9BZE0",
  "term_label": "negative regulation of transcription by RNA polymerase II"
}